diacylglycerol cholinephosphotransferase activity [GO:0004142] (molecular function) Relationships: is a type of CDP-alcohol phosphatidyltransferase activity [GO:0017169]; is part of CDP-choline pathway [GO:0006657] Definition: Catalysis of the reaction: CDP-choline + 1,2-diacylglycerol = CMP + a phosphatidylcholine. Sources: EC:2.7.8.2, RHEA:32939 Also known as: 1-alkyl-2-acetyl-m-glycerol:CDPcholine choline phosphotransferase activity, 1-alkyl-2-acetyl-sn-glycerol cholinephosphotransferase activity, 1-alkyl-2-acetylglycerol cholinephosphotransferase activity, CDP-choline diglyceride phosphotransferase activity, CDP-choline:1,2-diacylglycerol cholinephosphotransferase activity, CPT, alkylacylglycerol choline phosphotransferase activity, alkylacylglycerol cholinephosphotransferase activity, cholinephosphotransferase activity, cytidine diphosphocholine glyceride transferase activity, cytidine diphosphorylcholine diglyceride transferase activity, diacylglycerol choline phosphotransferase activity, phosphocholine diacylglyceroltransferase activity, phosphorylcholine--glyceride transferase activity, sn-1,2-diacylglycerol cholinephosphotransferase activity